CCACCA tRNA nucleotidyltransferase activity [GO:0160016] (molecular function) Relationships: is a type of cytidylyltransferase activity [GO:0070567]; is a type of catalytic activity, acting on a tRNA [GO:0140101] Definition: Catalysis of the reaction: a tRNA with a 3' CCA end + 2 CTP + ATP = a tRNA with a 3' CCACCA end + 3 diphosphate. References: PMID:22076379 Sources: RHEA:76235